NAD transmembrane transporter activity [GO:0051724] (molecular function) Definition: Enables the transfer of NAD from one side of a membrane to the other. Also known as: NAD (oxidized) transporter activity, NAD (reduced) transporter activity, NAD+ transporter activity, NADH transporter activity, nicotinamide adenine dinucleotide transmembrane transporter activity, oxidized NAD transporter activity, oxidized nicotinamide adenine dinucleotide transmembrane transporter activity, reduced NAD transporter activity, reduced nicotinamide adenine dinucleotide transmembrane transporter activity, NAD transporter activity Relationships: is a type of adenine nucleotide transmembrane transporter activity [GO:0000295]; BFO_0000050 NAD transmembrane transport [GO:0035352] Sources: GOC:TermGenie Note: NAD carrier